{
  "gene_symbol": "ZDHHC2",
  "gene_name": "Palmitoyltransferase ZDHHC2",
  "term_id": "GO:0016188",
  "gene": "UniProtKB:Q9UIJ5",
  "term_label": "synaptic vesicle maturation"
}